{
  "gene_name": "Tyrosyl-DNA phosphodiesterase 2",
  "term_label": "5'-tyrosyl-DNA phosphodiesterase activity",
  "gene": "UniProtKB:O95551",
  "gene_symbol": "TDP2",
  "term_id": "GO:0070260"
}